methanophenazine reducing hydrogenase complex [GO:0044679] (cellular component) Definition: A protein complex which catalyzes the conversion of methanophenazine and hydrogen to form dihydromethanophenazine. This typically consists of three polypeptides. Relationships: is a type of GO:1990204 References: PMID:9555882 Sources: GOC:mengo_curators